negative regulation of vesicle fusion with Golgi apparatus [GO:0106215] (biological process) Relationships: is_a GO:0031339; is a type of regulation of vesicle fusion with Golgi apparatus [GO:0106214]; negatively regulates vesicle fusion with Golgi apparatus [GO:0048280] References: PMID:26195667 Sources: GOC:se Definition: Any process that stops, prevents or reduces the frequency, rate or extent of vesicle fustion with Golgi apparatus.